sinapoylglucose-choline O-sinapoyltransferase activity [GO:0047202] (MF) Also known as: 1-O-(4-hydroxy-3,5-dimethoxycinnamoyl)-beta-D-glucose:choline 1-O-(4-hydroxy-3,5-dimethoxycinnamoyl)transferase activity, sinapine synthase activity Definition: Catalysis of the reaction: 1-O-sinapoyl-beta-D-glucose + choline = O-sinapoylcholine + D-glucose. Relationships: is a type of O-sinapoyltransferase activity [GO:0016753] Sources: EC:2.3.1.91, RHEA:12024